{
  "term_id": "GO:0005634",
  "term_label": "nucleus",
  "gene": "UniProtKB:Q6ZN01",
  "gene_name": "MEF2-activating motif and SAP domain-containing transcriptional regulator",
  "gene_symbol": "MAMSTR"
}